{
  "term_id": "GO:0052735",
  "gene_symbol": "METTL2B",
  "gene": "UniProtKB:Q6P1Q9",
  "gene_name": "tRNA N(3)-methylcytidine methyltransferase METTL2B",
  "term_label": "tRNA (cytidine-3-)-methyltransferase activity"
}